{
  "term_id": "GO:0043005",
  "gene": "UniProtKB:Q494W8",
  "gene_name": "CHRNA7-FAM7A fusion protein",
  "gene_symbol": "CHRFAM7A",
  "term_label": "neuron projection"
}